{
  "term_label": "Unknown cellular component",
  "gene_symbol": "IGHV1-58",
  "gene_name": "Immunoglobulin heavy variable 1-58",
  "term_id": "UNKNOWN:0003",
  "gene": "UniProtKB:A0A0C4DH39"
}